DNA topoisomerase III-beta-TDRD3 complex [GO:0140225] (cellular component) Definition: A protein complex that has DNA topoisomerase type I and RNA topoisomerase activities. Relationships: is a type of protein-containing complex [GO:0032991] Also known as: Top3-beta-TDRD3 complex References: PMID:23912945, PMID:28176834 Sources: GOC:lnp